{
  "term_label": "RNA polymerase II cis-regulatory region sequence-specific DNA binding",
  "gene_name": "Transcription factor Maf",
  "term_id": "GO:0000978",
  "gene": "UniProtKB:O75444",
  "gene_symbol": "MAF"
}